{
  "gene_symbol": "ZUP1",
  "gene_name": "Zinc finger-containing ubiquitin peptidase 1",
  "term_label": "transcription cis-regulatory region binding",
  "gene": "UniProtKB:Q96AP4",
  "term_id": "GO:0000976"
}